{
  "term_label": "sodium ion export across plasma membrane",
  "term_id": "GO:0036376",
  "gene_name": "Potassium-transporting ATPase subunit beta",
  "gene_symbol": "ATP4B",
  "gene": "UniProtKB:P51164"
}